{
  "term_id": "GO:0005634",
  "gene_symbol": "ONECUT1",
  "gene": "UniProtKB:Q9UBC0",
  "gene_name": "Hepatocyte nuclear factor 6",
  "term_label": "nucleus"
}